cargo receptor complex [GO:0062137] (cellular component) Subtypes: low-density lipoprotein receptor complex [GO:0062136] Relationships: is_a membrane protein complex [GO:0098796] References: PMID:27903609 Definition: Any protein complex that is part of a membrane and which functions as a cargo receptor.